{
  "term_label": "Unknown cellular component",
  "term_id": "UNKNOWN:0003",
  "gene": "UniProtKB:P58005",
  "gene_name": "Sestrin-3",
  "gene_symbol": "SESN3"
}